ceramide cholinephosphotransferase activity [GO:0047493] (molecular function) Relationships: is a type of GO:0016780 Sources: EC:2.7.8.3, RHEA:16273 Also known as: CDP-choline:N-acylsphingosine cholinephosphotransferase activity, phosphorylcholine-ceramide transferase activity Definition: Catalysis of the reaction: CDP-choline + ceramide = CMP + H+ + sphingomyelin.